{
  "gene_name": "Zinc finger protein 624",
  "term_label": "DNA-binding transcription factor activity, RNA polymerase II-specific",
  "term_id": "GO:0000981",
  "gene_symbol": "ZNF624",
  "gene": "UniProtKB:Q9P2J8"
}